{
  "gene": "UniProtKB:Q16828",
  "gene_name": "Dual specificity protein phosphatase 6",
  "term_label": "MAP kinase tyrosine/serine/threonine phosphatase activity",
  "gene_symbol": "DUSP6",
  "term_id": "GO:0017017"
}